{
  "gene_symbol": "PYCR3",
  "gene_name": "Pyrroline-5-carboxylate reductase 3",
  "term_id": "GO:0055129",
  "gene": "UniProtKB:Q53H96",
  "term_label": "L-proline biosynthetic process"
}